{
  "gene_name": "Ephrin-B3",
  "term_label": "presynaptic membrane",
  "gene_symbol": "EFNB3",
  "term_id": "GO:0042734",
  "gene": "UniProtKB:Q15768"
}